annulate lamellae [GO:0005642] (cellular component) Relationships: is a type of GO:0016020; is part of GO:0042175 References: PMID:12631728 Definition: Stacks of endoplasmic reticulum (ER) membranes containing a high density of nuclear pores, thought to form from excess nuclear membrane components, that have been described in a number of different cells. Annulate lamellar membranes are continuous with and embedded within the ER.